{
  "gene_name": "DNA dC-dU-editing enzyme APOBEC-3B",
  "term_id": "GO:0004126",
  "gene_symbol": "APOBEC3B",
  "term_label": "cytidine deaminase activity",
  "gene": "UniProtKB:Q9UH17"
}